{
  "gene": "UniProtKB:Q9UKV5",
  "gene_name": "E3 ubiquitin-protein ligase AMFR",
  "term_label": "ubiquitin protein ligase activity",
  "gene_symbol": "AMFR",
  "term_id": "GO:0061630"
}